regulation of mismatch repair [GO:0032423] (biological process) Sources: GOC:vk Relationships: is a type of regulation of DNA repair [GO:0006282]; regulates mismatch repair [GO:0006298] Subtypes: negative regulation of mismatch repair [GO:0032424], positive regulation of mismatch repair [GO:0032425] Definition: Any process that modulates the frequency, rate or extent of mismatch repair.